{
  "term_label": "nucleus",
  "gene_symbol": "JDP2",
  "gene_name": "Jun dimerization protein 2",
  "term_id": "GO:0005634",
  "gene": "UniProtKB:Q8WYK2"
}